{
  "gene": "UniProtKB:Q7Z6K3",
  "gene_symbol": "PTAR1",
  "term_id": "GO:0004663",
  "gene_name": "Protein prenyltransferase alpha subunit repeat-containing protein 1",
  "term_label": "Rab geranylgeranyltransferase activity"
}